regulation of biosynthetic process of antibacterial peptides active against Gram-positive bacteria [GO:0002816] (BP) Relationships: is a type of regulation of antibacterial peptide biosynthetic process [GO:0002808]; RO_0002211 biosynthetic process of antibacterial peptides active against Gram-positive bacteria [GO:0002815] Subtypes: negative regulation of biosynthetic process of antibacterial peptides active against Gram-positive bacteria [GO:0002817], positive regulation of biosynthetic process of antibacterial peptides active against Gram-positive bacteria [GO:0006965] Sources: GOC:add Definition: Any process that modulates the frequency, rate, or extent of biosynthesis of antibacterial peptides active against Gram-positive bacteria.